{
  "gene_name": "Glutamyl-tRNA(Gln) amidotransferase subunit C, mitochondrial",
  "gene": "UniProtKB:O43716",
  "gene_symbol": "GATC",
  "term_label": "glutaminyl-tRNAGln biosynthesis via transamidation",
  "term_id": "GO:0070681"
}